{
  "gene_name": "Phosphatidylinositol 3-kinase catalytic subunit type 3",
  "gene_symbol": "PIK3C3",
  "term_label": "phosphatidylinositol-3-phosphate biosynthetic process",
  "gene": "UniProtKB:Q8NEB9",
  "term_id": "GO:0036092"
}